{
  "gene_name": "Adenomatous polyposis coli protein 2",
  "gene_symbol": "APC2",
  "term_label": "cell migration",
  "gene": "UniProtKB:O95996",
  "term_id": "GO:0016477"
}